{
  "gene_name": "Transcription factor HES-3",
  "term_label": "RNA polymerase II cis-regulatory region sequence-specific DNA binding",
  "gene_symbol": "HES3",
  "gene": "UniProtKB:Q5TGS1",
  "term_id": "GO:0000978"
}